{
  "term_id": "GO:0000978",
  "gene": "UniProtKB:Q5T1R4",
  "gene_name": "Transcription factor HIVEP3",
  "gene_symbol": "HIVEP3",
  "term_label": "RNA polymerase II cis-regulatory region sequence-specific DNA binding"
}